{
  "gene_name": "Eukaryotic translation initiation factor 4E type 2",
  "term_id": "GO:0016281",
  "gene": "UniProtKB:O60573",
  "gene_symbol": "EIF4E2",
  "term_label": "eukaryotic translation initiation factor 4F complex"
}